{
  "gene_symbol": "STX5",
  "gene": "UniProtKB:Q13190",
  "term_label": "vesicle docking",
  "gene_name": "Syntaxin-5",
  "term_id": "GO:0048278"
}